histone H3 acetyltransferase activity [GO:0010484] (molecular function) Definition: Catalysis of the reaction: acetyl-CoA + histone H3 = CoA + acetyl-histone H3. References: PMID:19056256 Also known as: H3 histone acetylase activity, H3 histone acetyltransferase activity Relationships: is a type of GO:0004402 Subtypes: GO:0032931, GO:0036408, histone H3K9 acetyltransferase activity [GO:0043992], histone H3K18 acetyltransferase activity [GO:0043993], histone H3K23 acetyltransferase activity [GO:0043994], histone H3K4 acetyltransferase activity [GO:0044016], GO:0044017, histone H3K36 acetyltransferase activity [GO:0044018], histone H3K122 acetyltransferase activity [GO:0140908]